{
  "term_id": "GO:0005634",
  "gene_symbol": "CDK2AP2",
  "gene": "UniProtKB:O75956",
  "term_label": "nucleus",
  "gene_name": "Cyclin-dependent kinase 2-associated protein 2"
}